organelle inheritance [GO:0048308] (biological process) Subtypes: mitochondrion inheritance [GO:0000001], GO:0000011, plastid inheritance [GO:0009665], peroxisome inheritance [GO:0045033], endoplasmic reticulum inheritance [GO:0048309], Golgi inheritance [GO:0048313] Definition: The partitioning of organelles between daughter cells at cell division. Sources: GOC:jid Relationships: is a type of organelle organization [GO:0006996]